{
  "term_label": "sperm axoneme assembly",
  "gene_symbol": "SPAG6",
  "term_id": "GO:0007288",
  "gene": "UniProtKB:O75602",
  "gene_name": "Sperm-associated antigen 6"
}